{
  "gene": "UniProtKB:Q9BT40",
  "gene_symbol": "INPP5K",
  "term_label": "negative regulation of phosphatidylinositol 3-kinase/protein kinase B signal transduction",
  "gene_name": "Inositol polyphosphate 5-phosphatase K",
  "term_id": "GO:0051898"
}